{
  "term_id": "GO:0042923",
  "term_label": "neuropeptide binding",
  "gene_name": "Probable G-protein coupled receptor 149",
  "gene": "UniProtKB:Q86SP6",
  "gene_symbol": "GPR149"
}